{
  "gene_name": "Nucleoporin NUP188",
  "term_label": "RNA export from nucleus",
  "gene": "UniProtKB:Q5SRE5",
  "gene_symbol": "NUP188",
  "term_id": "GO:0006405"
}